anatomical structure maturation [GO:0071695] (biological process) Sources: GOC:mah Subtypes: blood vessel maturation [GO:0001955], fruit ripening [GO:0009835], GO:0021578, medulla oblongata maturation [GO:0021582], GO:0021586, cerebellum maturation [GO:0021590], GO:0021626, GO:0021682, cerebellar granular layer maturation [GO:0021686], cerebellar molecular layer maturation [GO:0021690], cerebellar Purkinje cell layer maturation [GO:0021691], cerebellar cortex maturation [GO:0021699], locus ceruleus maturation [GO:0021706], GO:0021717, superior olivary nucleus maturation [GO:0021722], midbrain-hindbrain boundary maturation [GO:0021732], dorsal motor nucleus of vagus nerve maturation [GO:0035761], cell maturation [GO:0048469], animal organ maturation [GO:0048799], hair follicle maturation [GO:0048820], ganglion maturation [GO:0061553], secretory granule maturation [GO:0061792], olfactory placode maturation [GO:0071700] Relationships: is_a developmental maturation [GO:0021700]; is part of anatomical structure development [GO:0048856] Definition: A developmental process, independent of morphogenetic (shape) change, that is required for an anatomical structure to attain its fully functional state.